{
  "gene": "UniProtKB:Q9UPQ3",
  "term_label": "Unknown biological process",
  "gene_name": "Arf-GAP with GTPase, ANK repeat and PH domain-containing protein 1",
  "gene_symbol": "AGAP1",
  "term_id": "UNKNOWN:0002"
}